regulation of salicylic acid metabolic process [GO:0010337] (biological process) Definition: Any process that modulates the frequency, rate or extent of the chemical reactions and pathways involving salicylic acid. References: PMID:14765119 Relationships: is a type of regulation of ketone metabolic process [GO:0010565]; is a type of regulation of small molecule metabolic process [GO:0062012]; regulates GO:0009696 Also known as: regulation of salicylic acid metabolism Subtypes: regulation of salicylic acid biosynthetic process [GO:0080142]